heme C catabolic process [GO:0046163] (biological process) Relationships: is a type of heme catabolic process [GO:0042167] Definition: The chemical reactions and pathways resulting in the breakdown of heme C, a derivative of heme found in cytochromes c, b4, and f. Sources: GOC:curators Also known as: haem C catabolic process, haem C catabolism, heme C breakdown, heme C catabolism, heme C degradation